{
  "gene_name": "tRNA (adenine(58)-N(1))-methyltransferase, mitochondrial",
  "gene": "UniProtKB:Q9BVS5",
  "gene_symbol": "TRMT61B",
  "term_id": "GO:0160107",
  "term_label": "tRNA (adenine(58)-N1)-methyltransferase activity"
}